{
  "gene": "UniProtKB:Q96FK6",
  "gene_name": "WD repeat-containing protein 89",
  "term_id": "UNKNOWN:0002",
  "term_label": "Unknown biological process",
  "gene_symbol": "WDR89"
}